{
  "gene": "UniProtKB:P01210",
  "gene_symbol": "PENK",
  "gene_name": "Proenkephalin-A",
  "term_id": "GO:0043679",
  "term_label": "axon terminus"
}